{
  "term_id": "GO:0005765",
  "term_label": "lysosomal membrane",
  "gene_name": "HLA class II histocompatibility antigen, DP alpha 1 chain",
  "gene": "UniProtKB:P20036",
  "gene_symbol": "HLA-DPA1"
}